{
  "gene": "UniProtKB:Q9UHP3",
  "gene_symbol": "USP25",
  "gene_name": "Ubiquitin carboxyl-terminal hydrolase 25",
  "term_label": "cytosol",
  "term_id": "GO:0005829"
}